ultradian rhythm [GO:0007624] (biological process) Subtypes: defecation rhythm [GO:0035882] References: PMID:19708721 Sources: GOC:jl Relationships: is a type of rhythmic process [GO:0048511] Definition: The specific actions or reactions of an organism that recur with a regularity more frequent than every 24 hours.